{
  "gene_symbol": "TEX19",
  "gene": "UniProtKB:Q8NA77",
  "term_label": "spermatogenesis",
  "term_id": "GO:0007283",
  "gene_name": "Testis-expressed protein 19"
}